{
  "gene": "UniProtKB:P48047",
  "gene_name": "ATP synthase subunit O, mitochondrial",
  "term_label": "proton-transporting ATP synthase activity, rotational mechanism",
  "term_id": "GO:0046933",
  "gene_symbol": "ATP5PO"
}